{
  "term_label": "phosphatidylethanolamine N-methyltransferase activity",
  "term_id": "GO:0004608",
  "gene": "UniProtKB:Q9UBM1",
  "gene_name": "Phosphatidylethanolamine N-methyltransferase",
  "gene_symbol": "PEMT"
}